oxalomalate lyase activity [GO:0050204] (molecular function) Relationships: is a type of GO:0016833 Also known as: 3-oxalomalate glyoxylate-lyase (oxaloacetate-forming), 3-oxalomalate glyoxylate-lyase activity Sources: EC:4.1.3.13, RHEA:22032 Definition: Catalysis of the reaction: 3-oxalomalate = glyoxylate + oxaloacetate.